{
  "gene": "UniProtKB:Q8WWR8",
  "gene_name": "Sialidase-4",
  "term_label": "membrane",
  "term_id": "GO:0016020",
  "gene_symbol": "NEU4"
}